{
  "term_label": "brahma complex",
  "gene": "UniProtKB:Q12824",
  "term_id": "GO:0035060",
  "gene_name": "SWI_SNF-related matrix-associated actin-dependent regulator of chromatin subfamily B member 1",
  "gene_symbol": "SMARCB1"
}